{
  "term_label": "nucleus",
  "gene_name": "Zinc finger protein 525",
  "gene_symbol": "ZNF525",
  "gene": "UniProtKB:Q8N782",
  "term_id": "GO:0005634"
}